basolateral plasma membrane [GO:0016323] (cellular component) Definition: The region of the plasma membrane that includes the basal end and sides of the cell. Often used in reference to animal polarized epithelial membranes, where the basal membrane is the part attached to the extracellular matrix, or in plant cells, where the basal membrane is defined with respect to the zygotic axis. Sources: GOC:go_curators Relationships: is a type of plasma membrane region [GO:0098590]; is part of GO:0009925